mucilage biosynthetic process involved in seed coat development [GO:0048354] (biological process) Definition: The chemical reactions and pathways resulting in the formation of mucilage that occur as part of seed coat development; mucilage is normally synthesized during seed coat development. Sources: GOC:dph, GOC:jid, GOC:tb Also known as: mucilage anabolism during seed coat development, mucilage formation during seed coat development, mucilage synthesis during seed coat development, mucilage biosynthetic process during seed coat development Relationships: is a type of GO:0010192; is part of seed coat development [GO:0010214]